{
  "gene_symbol": "RAET1G",
  "term_label": "extracellular space",
  "gene": "UniProtKB:Q6H3X3",
  "term_id": "GO:0005615",
  "gene_name": "UL-16 binding protein 5"
}